histone H3K14 acetyltransferase activity [GO:0036408] (molecular function) Note: Comment: Note that the residue position corresponds to the canonical human H3 histone (UniProtKB:P84243); this residue is conserved across all eukaryotes. Residue 1 is the first residue following removal of the initiating Methionine (Met). Note that each histone is encoded by multiple genes, and sequences may vary across different genes within an organism. Also known as: histone H3-K14 acetyltransferase activity, histone acetylase activity (H3-K14 specific), histone acetyltransferase activity (H3-K14 specific), histone lysine N-acetyltransferase activity (H3-K14 specific) References: PMID:18552846, PMID:19056256, PMID:21289066 Sources: GOC:vw Definition: Catalysis of the reaction: acetyl-CoA + histone H3 L-lysine (position 14) = CoA + histone H3 N6-acetyl-L-lysine (position 14). Relationships: is a type of GO:0010484